acetyl-CoA:oxalate CoA-transferase [GO:0036412] (molecular function) Relationships: is a type of CoA-transferase activity [GO:0008410] References: PMID:23935849 Sources: GOC:imk Definition: Catalysis of the reaction: acetyl-CoA + oxalate = acetate + oxalyl-CoA.